{
  "term_label": "Unknown cellular component",
  "term_id": "UNKNOWN:0003",
  "gene_name": "Olfactory receptor 5H1",
  "gene_symbol": "OR5H1",
  "gene": "UniProtKB:A6NKK0"
}